{
  "term_id": "GO:0005884",
  "gene": "UniProtKB:P57737",
  "gene_symbol": "CORO7",
  "gene_name": "Coronin-7",
  "term_label": "actin filament"
}